{
  "gene_name": "Latent-transforming growth factor beta-binding protein 4",
  "gene_symbol": "LTBP4",
  "term_label": "extracellular matrix",
  "gene": "UniProtKB:Q8N2S1",
  "term_id": "GO:0031012"
}